regulation of lipid biosynthetic process [GO:0046890] (BP) Definition: Any process that modulates the frequency, rate or extent of the chemical reactions and pathways resulting in the formation of lipids. Sources: GOC:ai Subtypes: regulation of juvenile hormone biosynthetic process [GO:0007557], regulation of abscisic acid biosynthetic process [GO:0010115], regulation of gibberellin biosynthetic process [GO:0010371], regulation of triglyceride biosynthetic process [GO:0010866], regulation of fatty acid biosynthetic process [GO:0042304], positive regulation of lipid biosynthetic process [GO:0046889], regulation of steroid biosynthetic process [GO:0050810], negative regulation of lipid biosynthetic process [GO:0051055], regulation of phospholipid biosynthetic process [GO:0071071], regulation of sphingolipid biosynthetic process [GO:0090153], regulation of retinoic acid biosynthetic process [GO:1900052], regulation of diacylglycerol biosynthetic process [GO:1900480], regulation of butyryl-CoA catabolic process to butanol [GO:1900497], regulation of emericellamide biosynthetic process [GO:1900658], GO:1900947, regulation of ent-pimara-8(14),15-diene biosynthetic process [GO:1901542], regulation of wax biosynthetic process [GO:1904276], regulation of phytol biosynthetic process [GO:1904963] Relationships: is a type of regulation of biosynthetic process [GO:0009889]; is a type of regulation of lipid metabolic process [GO:0019216]; regulates GO:0008610 Also known as: regulation of lipid anabolism, regulation of lipid biosynthesis, regulation of lipid formation, regulation of lipid synthesis, regulation of lipogenesis